{
  "term_label": "autophagosome maturation",
  "gene_name": "Ectopic P granules protein 5 homolog",
  "gene": "UniProtKB:Q9HCE0",
  "term_id": "GO:0097352",
  "gene_symbol": "EPG5"
}